{
  "gene_name": "Homeobox protein Hox-A3",
  "gene_symbol": "HOXA3",
  "term_id": "GO:0006357",
  "term_label": "regulation of transcription by RNA polymerase II",
  "gene": "UniProtKB:O43365"
}